{
  "gene": "UniProtKB:A6NEH8",
  "term_id": "UNKNOWN:0001",
  "term_label": "Unknown molecular function",
  "gene_name": "Putative uncharacterized protein encoded by ZNF503-AS2",
  "gene_symbol": "ZNF503-AS2"
}